regulation of monopolar cell growth [GO:0051513] (biological process) Definition: Any process that modulates the frequency, rate or extent of monopolar cell growth, polarized growth from one end of a cell. Sources: GOC:ai Relationships: is a type of GO:0051510; RO_0002211 monopolar cell growth [GO:0042814] Subtypes: negative regulation of monopolar cell growth [GO:0051514], positive regulation of monopolar cell growth [GO:0051515]